{
  "gene_name": "Ribose-5-phosphate isomerase",
  "gene_symbol": "RPIA",
  "term_id": "GO:0006014",
  "term_label": "D-ribose metabolic process",
  "gene": "UniProtKB:P49247"
}